{
  "gene_name": "Histone-binding protein RBBP7",
  "term_id": "GO:0042393",
  "term_label": "histone binding",
  "gene_symbol": "RBBP7",
  "gene": "UniProtKB:Q16576"
}